{
  "gene_name": "Circadian-associated transcriptional repressor",
  "term_label": "negative regulation of DNA-templated transcription",
  "term_id": "GO:0045892",
  "gene": "UniProtKB:Q8N365",
  "gene_symbol": "CIART"
}